{
  "term_id": "GO:0000151",
  "gene_symbol": "RNF144A",
  "term_label": "ubiquitin ligase complex",
  "gene_name": "E3 ubiquitin-protein ligase RNF144A",
  "gene": "UniProtKB:P50876"
}